viral DNA genome packaging, 3' extended cos packaging [GO:0098036] (biological process) Definition: The encapsulation of the viral DNA genome within the capsid, which proceeds via cleavage of the viral DNA at specific sites to produce 3' protruding ends. Relationships: is_a viral DNA genome packaging via site-specific sequence recognition [GO:0098035] Sources: GOC:bm